{
  "term_label": "acetoacetate-CoA ligase activity",
  "term_id": "GO:0030729",
  "gene_symbol": "AACS",
  "gene": "UniProtKB:Q86V21",
  "gene_name": "Acetoacetyl-CoA synthetase"
}